{
  "gene_name": "Transmembrane protein 254",
  "term_label": "Unknown cellular component",
  "gene_symbol": "TMEM254",
  "gene": "UniProtKB:Q8TBM7",
  "term_id": "UNKNOWN:0003"
}